{
  "term_label": "Unknown cellular component",
  "gene_symbol": "IKZF5",
  "term_id": "UNKNOWN:0003",
  "gene_name": "Zinc finger protein Pegasus",
  "gene": "UniProtKB:Q9H5V7"
}